{
  "gene_symbol": "NOX1",
  "term_id": "GO:0016175",
  "gene": "UniProtKB:Q9Y5S8",
  "gene_name": "NADPH oxidase 1",
  "term_label": "superoxide-generating NAD(P)H oxidase activity"
}